L-asparagine, sodium:proton antiporter activity [GO:0140831] (MF) References: PMID:10619430, PMID:11742981 Definition: Enables the transfer of a solute or solutes from one side of a membrane to the other according to the reaction: H+(in) + L-asparagine(out) + Na+(out) = H+(out) + L-asparagine(in) + Na+(in). Relationships: is a type of GO:0015182; is a type of sodium:proton antiporter activity [GO:0015385]; is a type of amino acid:monoatomic cation antiporter activity [GO:0140848]